{
  "gene_name": "Homeobox protein Hox-A6",
  "gene_symbol": "HOXA6",
  "term_id": "GO:0000981",
  "gene": "UniProtKB:P31267",
  "term_label": "DNA-binding transcription factor activity, RNA polymerase II-specific"
}